lytic vacuole organization [GO:0080171] (biological process) Subtypes: lysosome organization [GO:0007040] Relationships: is a type of vacuole organization [GO:0007033] References: PMID:20729380 Also known as: lytic vacuole organisation, lytic vacuolar assembly, lytic vacuole biogenesis, lytic vacuole organization and biogenesis Definition: A process that is carried out at the cellular level which results in the assembly, arrangement of constituent parts, or disassembly of a lytic vacuole.